{
  "term_label": "cytosol",
  "gene": "UniProtKB:Q86YL5",
  "gene_symbol": "TDRP",
  "gene_name": "Testis development-related protein",
  "term_id": "GO:0005829"
}